{
  "gene_name": "Transcription cofactor vestigial-like protein 2",
  "term_label": "nucleus",
  "term_id": "GO:0005634",
  "gene_symbol": "VGLL2",
  "gene": "UniProtKB:Q8N8G2"
}